{
  "gene_symbol": "CHCT1",
  "gene_name": "CHD1 helical C-terminal domain containing protein 1",
  "term_label": "Unknown molecular function",
  "gene": "UniProtKB:Q86WR6",
  "term_id": "UNKNOWN:0001"
}